calcium channel inhibitor activity [GO:0019855] (molecular function) Relationships: is a type of calcium channel regulator activity [GO:0005246]; is a type of ion channel inhibitor activity [GO:0008200]; negatively regulates GO:0005262 Definition: Binds to and stops, prevents, or reduces the activity of a calcium channel. Sources: GOC:mah